{
  "gene": "UniProtKB:O75251",
  "gene_name": "NADH dehydrogenase [ubiquinone] iron-sulfur protein 7, mitochondrial",
  "term_label": "aerobic respiration",
  "gene_symbol": "NDUFS7",
  "term_id": "GO:0009060"
}